{
  "gene_name": "Vitamin K epoxide reductase complex subunit 1",
  "gene_symbol": "VKORC1",
  "term_id": "GO:0047057",
  "term_label": "vitamin-K-epoxide reductase (warfarin-sensitive) activity",
  "gene": "UniProtKB:Q9BQB6"
}